{
  "term_label": "nitrate metabolic process",
  "term_id": "GO:0042126",
  "gene": "UniProtKB:Q5VT66",
  "gene_name": "Mitochondrial amidoxime-reducing component 1",
  "gene_symbol": "MTARC1"
}